{
  "gene_symbol": "TMED5",
  "gene_name": "Transmembrane emp24 domain-containing protein 5",
  "gene": "UniProtKB:Q9Y3A6",
  "term_id": "GO:0005783",
  "term_label": "endoplasmic reticulum"
}